{
  "term_label": "Unknown molecular function",
  "gene_name": "Putative uncharacterized protein ENSP00000383407",
  "term_id": "UNKNOWN:0001",
  "gene_symbol": "A8MT66",
  "gene": "UniProtKB:A8MT66"
}